{
  "gene": "UniProtKB:Q8IVF4",
  "term_id": "GO:0060294",
  "gene_name": "Dynein axonemal heavy chain 10",
  "term_label": "cilium movement involved in cell motility",
  "gene_symbol": "DNAH10"
}